{
  "gene": "UniProtKB:P02765",
  "gene_symbol": "AHSG",
  "term_label": "acute-phase response",
  "term_id": "GO:0006953",
  "gene_name": "Alpha-2-HS-glycoprotein"
}